positive regulation of estrogen secretion [GO:2000863] (biological process) Sources: GOC:sl Also known as: positive regulation of oestrogen secretion Definition: Any process that activates or increases the frequency, rate or extent of estrogen secretion. Relationships: is_a positive regulation of steroid hormone secretion [GO:2000833]; is a type of regulation of estrogen secretion [GO:2000861]; positively regulates GO:0035937